{
  "gene_symbol": "FCER1G",
  "term_label": "immunoglobulin mediated immune response",
  "gene": "UniProtKB:P30273",
  "gene_name": "High affinity immunoglobulin epsilon receptor subunit gamma",
  "term_id": "GO:0016064"
}